{
  "term_label": "cytoplasm",
  "gene_symbol": "DAPK1",
  "term_id": "GO:0005737",
  "gene_name": "Death-associated protein kinase 1",
  "gene": "UniProtKB:P53355"
}